{
  "gene_name": "Nuclear receptor subfamily 4 group A member 1",
  "term_label": "regulation of transcription by RNA polymerase II",
  "gene_symbol": "NR4A1",
  "gene": "UniProtKB:P22736",
  "term_id": "GO:0006357"
}